{
  "gene_symbol": "CARD9",
  "term_id": "GO:0050776",
  "term_label": "regulation of immune response",
  "gene": "UniProtKB:Q9H257",
  "gene_name": "Caspase recruitment domain-containing protein 9"
}